intracellular cobalt ion homeostasis [GO:0006877] (biological process) Relationships: is a type of GO:0030003; is a type of inorganic ion homeostasis [GO:0098771] Definition: A homeostatic process involved in the maintenance of a steady state level of cobalt (Co2+) ions within a cell. Also known as: cobalt homeostasis, cellular cobalt ion homeostasis Sources: GOC:ai, GOC:mah